2-hydroxyisoflavanone dehydratase activity [GO:0033987] (molecular function) Relationships: is a type of hydro-lyase activity [GO:0016836] Sources: EC:4.2.1.105 Definition: Catalysis of the reactions: (2R,3S)-2,4',7-trihydroxyisoflavanone = daidzein + H+ + H2O, and 2-hydroxy-2,3-dihydrogenistein = genistein + H+ + H2O. Also known as: 2,7,4'-trihydroxyisoflavanone hydro-lyase (daidzein-forming) activity, 2,7,4'-trihydroxyisoflavanone hydro-lyase activity